{
  "gene_symbol": "PTGIS",
  "term_id": "UNKNOWN:0003",
  "term_label": "Unknown cellular component",
  "gene": "UniProtKB:Q16647",
  "gene_name": "Prostacyclin synthase"
}